cranial ganglion formation [GO:0061560] (biological process) Sources: GOC:dph Relationships: is a type of GO:0061554; BFO_0000050 cranial ganglion morphogenesis [GO:0061559] Subtypes: trigeminal ganglion formation [GO:0061561] Definition: The process that gives rise to a cranial ganglion. This process pertains to the initial formation of a structure from unspecified parts. Also known as: cranial ganglia formation